{
  "term_id": "GO:0072657",
  "term_label": "protein localization to membrane",
  "gene_symbol": "TM9SF4",
  "gene": "UniProtKB:Q92544",
  "gene_name": "Transmembrane 9 superfamily member 4"
}